spermidine acetylation [GO:0032918] (biological process) Relationships: is a type of spermidine metabolic process [GO:0008216]; is a type of polyamine acetylation [GO:0032917] Definition: The modification of spermidine by addition of acetyl groups. Sources: GOC:mlg